{
  "gene": "UniProtKB:Q9GZP0",
  "term_label": "platelet-derived growth factor receptor signaling pathway",
  "gene_symbol": "PDGFD",
  "gene_name": "Platelet-derived growth factor D",
  "term_id": "GO:0048008"
}